branching involved in lymph vessel morphogenesis [GO:0060854] (biological process) Relationships: is a type of branching morphogenesis of an epithelial tube [GO:0048754]; is part of lymphangiogenesis [GO:0001946] Definition: The process of the coordinated growth and sprouting of lymph vessels giving rise to the organized lymphatic system. Also known as: patterning of lymph vessels Sources: GOC:dph, GOC:sdb_2009, GOC:tb